{
  "gene_symbol": "BRD8",
  "term_label": "NuA4 histone acetyltransferase complex",
  "term_id": "GO:0035267",
  "gene": "UniProtKB:Q9H0E9",
  "gene_name": "Bromodomain-containing protein 8"
}